{
  "term_label": "Atg12-Atg5-Atg16 complex",
  "gene_symbol": "ATG5",
  "gene": "UniProtKB:Q9H1Y0",
  "gene_name": "Autophagy protein 5",
  "term_id": "GO:0034274"
}